{
  "term_label": "clathrin-dependent endocytosis",
  "gene_name": "Clathrin coat assembly protein AP180",
  "term_id": "GO:0072583",
  "gene_symbol": "SNAP91",
  "gene": "UniProtKB:O60641"
}